phospholipid translocation [GO:0045332] (biological process) References: PMID:16452632, PMID:20043909, PMID:20302864 Sources: ISBN:0815316194 Regulation: regulated by regulation of phospholipid translocation [GO:0061091]; positively regulated by GO:0061092; negatively regulated by negative regulation of phospholipid translocation [GO:0061093] Also known as: flippase, phospholipid scrambling Definition: The movement of a phospholipid molecule from one leaflet of a membrane bilayer to the opposite leaflet. Note: Note that this term describes the transbilayer motion of individual phospholipid molecules, and should not be confused with 'phospholipid scrambling ; GO:0017121'. Subtypes: plasma membrane phospholipid scrambling [GO:0017121], GO:0140329, aminophospholipid translocation [GO:0140331] Relationships: is_a phospholipid transport [GO:0015914]; is a type of lipid translocation [GO:0034204]